positive regulation of antigen processing and presentation via MHC class Ib [GO:0002594] (biological process) Subtypes: GO:0002597, positive regulation of antigen processing and presentation of lipid antigen via MHC class Ib [GO:0002600] Also known as: up regulation of antigen processing and presentation via MHC class Ib, up-regulation of antigen processing and presentation via MHC class Ib, upregulation of antigen processing and presentation via MHC class Ib, activation of antigen processing and presentation via MHC class Ib, stimulation of antigen processing and presentation via MHC class Ib Relationships: is_a positive regulation of antigen processing and presentation [GO:0002579]; is a type of GO:0002592; positively regulates antigen processing and presentation via MHC class Ib [GO:0002475] Definition: Any process that activates or increases the frequency, rate, or extent of antigen processing and presentation of antigen via MHC class Ib. Sources: GOC:add